{
  "gene_symbol": "GJA5",
  "term_id": "GO:0086044",
  "term_label": "atrial cardiac muscle cell to AV node cell communication by electrical coupling",
  "gene_name": "Gap junction alpha-5 protein",
  "gene": "UniProtKB:P36382"
}